{
  "gene_name": "5'-3' exonuclease PLD3",
  "term_id": "GO:0012505",
  "gene": "UniProtKB:Q8IV08",
  "gene_symbol": "PLD3",
  "term_label": "endomembrane system"
}